S bouton [GO:1990027] (cellular component) Definition: Synaptic bouton found in the ventral horn of the spinal cord. S boutons range in diameter from 0.5 to 8 um and contain spherical synaptic vesicles. Sources: NIF_Subcellular:nlx_subcell_100207 Relationships: is_a GO:0043195